histone H3K23 ubiquitin ligase activity [GO:0140234] (molecular function) Relationships: is_a histone H3 ubiquitin ligase activity [GO:0141055] Definition: Catalysis of the transfer of a ubiquitin molecule to histone 3 at the lysine-23 residue. Note: Comment: Note that the residue position corresponds to the canonical human H3 histone (UniProtKB:P84243); this residue is conserved across all eukaryotes. Residue 1 is the first residue following removal of the initiating Methionine (Met). Note that each histone is encoded by multiple genes, and sequences may vary across different genes within an organism. References: PMID:40680746